mannotetraose 2-alpha-N-acetylglucosaminyltransferase activity [GO:0047222] (molecular function) Definition: Catalysis of the reaction: 1,3-alpha-D-mannosyl-1,2-alpha-D-mannosyl-1,2-alpha-D-mannosyl-D-mannose + UDP-N-acetyl-D-glucosamine = 1,3-alpha-D-mannosyl-1,2-(N-acetyl-alpha-D-glucosaminyl-alpha-D-mannosyl)-1,2-alpha-D-mannosyl-D-mannose + UDP. Sources: EC:2.4.1.138, MetaCyc:2.4.1.138-RXN Also known as: UDP-N-acetyl-D-glucosamine:mannotetraose alpha-N-acetyl-D-glucosaminyltransferase activity, alpha-N-acetylglucosaminyltransferase activity, uridine diphosphoacetylglucosamine mannoside alpha1->2-alphacetylglucosaminyltransferase activity Relationships: is a type of acetylglucosaminyltransferase activity [GO:0008375]